progesterone secretion [GO:0042701] (biological process) Regulation: RO_0002211 by regulation of progesterone secretion [GO:2000870]; negatively regulated by GO:2000871; positively regulated by positive regulation of progesterone secretion [GO:2000872] Sources: GOC:jl, ISBN:0395825172 Definition: The regulated release of progesterone, a steroid hormone, by the corpus luteum of the ovary and by the placenta. Relationships: is a type of cellular process involved in reproduction in multicellular organism [GO:0022412]; is a type of ovulation cycle process [GO:0022602]; is a type of steroid hormone secretion [GO:0035929]; is part of luteinization [GO:0001553]